{
  "term_label": "3',5'-cyclic-GMP phosphodiesterase activity",
  "gene_symbol": "PDE2A",
  "gene": "UniProtKB:O00408",
  "gene_name": "cGMP-dependent 3',5'-cyclic phosphodiesterase",
  "term_id": "GO:0047555"
}